{
  "term_label": "Cul4-RING E3 ubiquitin ligase complex",
  "gene": "UniProtKB:Q5H9S7",
  "gene_name": "DDB1- and CUL4-associated factor 17",
  "term_id": "GO:0080008",
  "gene_symbol": "DCAF17"
}